regulation of myoblast differentiation [GO:0045661] (biological process) Definition: Any process that modulates the frequency, rate or extent of myoblast differentiation. A myoblast is a mononucleate cell type that, by fusion with other myoblasts, gives rise to the myotubes that eventually develop into skeletal muscle fibers. Relationships: is a type of regulation of cell differentiation [GO:0045595]; regulates myoblast differentiation [GO:0045445] Subtypes: negative regulation of myoblast differentiation [GO:0045662], positive regulation of myoblast differentiation [GO:0045663], regulation of cardiac muscle cell myoblast differentiation [GO:2000690] Sources: CL:0000056, GOC:go_curators, GOC:mtg_muscle